{
  "gene_name": "[Pyruvate dehydrogenase [acetyl-transferring]]-phosphatase 2, mitochondrial",
  "gene_symbol": "PDP2",
  "term_id": "GO:0005739",
  "gene": "UniProtKB:Q9P2J9",
  "term_label": "mitochondrion"
}